LinE complex assembly [GO:0062120] (biological process) References: PMID:30640914 Relationships: is a type of protein-containing complex assembly [GO:0065003]; is a type of GO:1903046; is part of linear element assembly [GO:0030999] Definition: The aggregation, arrangement and bonding together of a set of components during meiotic prophase to form a LinE complex, the protein complex that associates with chromatin to form linear elements in fission yeast. In S. pombe, the LinE complex contains four main structural components (Rec10, Rec25, Rec27, and Mug20) and other associated proteins.